{
  "term_label": "Unknown molecular function",
  "gene_name": "Receptor-type tyrosine-protein phosphatase-like N",
  "gene": "UniProtKB:Q16849",
  "gene_symbol": "PTPRN",
  "term_id": "UNKNOWN:0001"
}